{
  "gene": "UniProtKB:Q96EW2",
  "gene_symbol": "HSPBAP1",
  "gene_name": "HSPB1-associated protein 1",
  "term_label": "2-oxoglutarate-dependent dioxygenase activity",
  "term_id": "GO:0016706"
}